{
  "gene_symbol": "SF3B5",
  "term_label": "Unknown molecular function",
  "gene_name": "Splicing factor 3B subunit 5",
  "term_id": "UNKNOWN:0001",
  "gene": "UniProtKB:Q9BWJ5"
}